{
  "term_id": "GO:0007283",
  "gene_symbol": "SPMAP2",
  "gene_name": "Testicular haploid expressed gene protein",
  "term_label": "spermatogenesis",
  "gene": "UniProtKB:Q9P2T0"
}